{
  "term_label": "D-aspartate oxidase activity",
  "term_id": "GO:0008445",
  "gene_name": "D-aspartate oxidase",
  "gene_symbol": "DDO",
  "gene": "UniProtKB:Q99489"
}